{
  "gene_symbol": "HDGFL3",
  "term_label": "Unknown cellular component",
  "term_id": "UNKNOWN:0003",
  "gene": "UniProtKB:Q9Y3E1",
  "gene_name": "Hepatoma-derived growth factor-related protein 3"
}